pyruvate fermentation [GO:0019660] (biological process) Subtypes: pyruvate fermentation to acetate [GO:0019654], pyruvate fermentation to ethanol [GO:0019655], pyruvate fermentation to propionate [GO:0019657], GO:0034079, GO:0044813, pyruvate fermentation via PFL [GO:0044814] Sources: GOC:curators Also known as: glycolytic fermentation Relationships: is a type of pyruvate catabolic process [GO:0042867]; is part of fermentation [GO:0006113] Definition: The fermentation process resulting in the oxygen-independent conversion of pyruvate to reduced end products (e.g., lactate, ethanol, and acetate), accompanied by the concomitant oxidation of NADH to NAD.